diethyl 2-methyl-3-oxosuccinate reductase activity [GO:0047031] (molecular function) Definition: Catalysis of the reaction: diethyl (2R,3R)-2-methyl-3-hydroxysuccinate + NADP+ = diethyl 2-methyl-3-oxosuccinate + H+ + NADPH. Also known as: diethyl-(2R,3R)-2-methyl-3-hydroxysuccinate:NADP+ 3-oxidoreductase activity Sources: EC:1.1.1.229, RHEA:21008 Relationships: is a type of oxidoreductase activity, acting on the CH-OH group of donors, NAD or NADP as acceptor [GO:0016616]